{
  "gene_symbol": "MID1IP1",
  "term_label": "nucleus",
  "gene": "UniProtKB:Q9NPA3",
  "gene_name": "Mid1-interacting protein 1",
  "term_id": "GO:0005634"
}